{
  "gene_name": "SLAM family member 9",
  "gene_symbol": "SLAMF9",
  "term_label": "external side of plasma membrane",
  "gene": "UniProtKB:Q96A28",
  "term_id": "GO:0009897"
}